blood vessel endothelial cell differentiation [GO:0060837] (BP) Sources: GOC:dph, GOC:sdb_2009, GOC:tb Relationships: is a type of endothelial cell differentiation [GO:0045446]; is part of GO:0001568 Subtypes: arterial endothelial cell differentiation [GO:0060842], GO:0060843, cardiac blood vessel endothelial cell differentiation [GO:0060946] Regulation: regulated by regulation of blood vessel endothelial cell differentiation [GO:0110057]; positively regulated by positive regulation of blood vessel endothelial cell differentiation [GO:0110058]; negatively regulated by negative regulation of blood vessel endothelial cell differentiation [GO:0110059] Definition: The process in which a relatively unspecialized cell acquires specialized features of a blood vessel endothelial cell, a thin flattened cell that lines the inside surfaces of blood vessels.